{
  "gene_name": "Histone acetyltransferase KAT2A",
  "gene_symbol": "KAT2A",
  "term_label": "positive regulation of transcription by RNA polymerase II",
  "term_id": "GO:0045944",
  "gene": "UniProtKB:Q92830"
}